{
  "gene_symbol": "ZSCAN1",
  "gene": "UniProtKB:Q8NBB4",
  "gene_name": "Zinc finger and SCAN domain-containing protein 1",
  "term_id": "GO:0000981",
  "term_label": "DNA-binding transcription factor activity, RNA polymerase II-specific"
}